{
  "term_id": "GO:0008017",
  "gene_name": "Microtubule-associated protein 6",
  "gene": "UniProtKB:Q96JE9",
  "term_label": "microtubule binding",
  "gene_symbol": "MAP6"
}